release of sequestered calcium ion into cytosol by endoplasmic reticulum [GO:1903514] (BP) References: PMID:16402920 Sources: GOC:BHF, GOC:TermGenie, GOC:mtg_cardiac_conduct_nov11, GOC:rl, GO_REF:0000078 Relationships: is a type of GO:0051209 Subtypes: GO:0014808 Also known as: calcium ion transport from endoplasmic reticulum to cytosol Definition: The directed movement of calcium ion from endoplasmic reticulum to cytosol.